{
  "gene_name": "ATP-dependent RNA helicase DDX25",
  "term_id": "GO:0005634",
  "term_label": "nucleus",
  "gene_symbol": "DDX25",
  "gene": "UniProtKB:Q9UHL0"
}